{
  "term_id": "GO:0005829",
  "gene_symbol": "PLA2G4E",
  "gene": "UniProtKB:Q3MJ16",
  "term_label": "cytosol",
  "gene_name": "Cytosolic phospholipase A2 epsilon"
}